{
  "term_label": "male germ cell nucleus",
  "gene": "UniProtKB:P09430",
  "gene_name": "Spermatid nuclear transition protein 1",
  "gene_symbol": "TNP1",
  "term_id": "GO:0001673"
}